{
  "gene_symbol": "TMEM150C",
  "gene": "UniProtKB:B9EJG8",
  "term_id": "UNKNOWN:0001",
  "term_label": "Unknown molecular function",
  "gene_name": "Transmembrane protein 150C"
}